{
  "gene_symbol": "M1AP",
  "term_label": "spermatogenesis",
  "gene_name": "Meiosis 1 arrest protein",
  "term_id": "GO:0007283",
  "gene": "UniProtKB:Q8TC57"
}